L-arginine deiminase pathway [GO:0019546] (biological process) Relationships: is a type of L-arginine catabolic process [GO:0006527]; has part arginine deiminase activity [GO:0016990] Definition: The chemical reactions and pathways resulting in the breakdown of L-arginine into other compounds, including ornithine and CO2, using the enzyme arginine deiminase. Sources: GOC:mah, MetaCyc:ARGDEGRAD-PWY